{
  "term_id": "UNKNOWN:0001",
  "gene_symbol": "PRM3",
  "gene_name": "Protamine-3",
  "term_label": "Unknown molecular function",
  "gene": "UniProtKB:Q9NNZ6"
}